{
  "term_label": "regulation of T cell proliferation",
  "gene_symbol": "TNFSF18",
  "gene_name": "Tumor necrosis factor ligand superfamily member 18",
  "gene": "UniProtKB:Q9UNG2",
  "term_id": "GO:0042129"
}